{
  "gene_symbol": "SULT1A3",
  "term_id": "GO:0005737",
  "gene": "UniProtKB:P0DMM9",
  "term_label": "cytoplasm",
  "gene_name": "Sulfotransferase 1A3"
}